{
  "gene": "UniProtKB:A0PJZ0",
  "gene_name": "Putative ankyrin repeat domain-containing protein 20A5",
  "term_id": "UNKNOWN:0001",
  "gene_symbol": "ANKRD20A5P",
  "term_label": "Unknown molecular function"
}